{
  "gene": "UniProtKB:Q99665",
  "term_label": "receptor complex",
  "gene_symbol": "IL12RB2",
  "gene_name": "Interleukin-12 receptor subunit beta-2",
  "term_id": "GO:0043235"
}